{
  "gene_symbol": "CTNND2",
  "term_id": "GO:0014069",
  "gene": "UniProtKB:Q9UQB3",
  "term_label": "postsynaptic density",
  "gene_name": "Catenin delta-2"
}